phosphodiesterase I activity [GO:0004528] (molecular function) Also known as: phosphodiesterase activity, 5' nucleotide phosphodiesterase/alkaline phosphodiesterase I activity, 5'-NPDase activity, 5'-PDE activity, 5'-PDase activity, 5'-exonuclease activity, 5'-nucleotide phosphodiesterase activity, 5'-phosphodiesterase activity, 5'NPDE activity, PDE I activity, alkaline phosphodiesterase activity, exonuclease I activity, nucleotide pyrophosphatase/phosphodiesterase I activity, oligonucleate 5'-nucleotidohydrolase activity, orthophosphoric diester phosphohydrolase activity Sources: EC:3.1.4.1 Regulation: positively regulated by positive regulation of phosphodiesterase I activity [GO:1902800] Definition: Catalysis of the sequential hydrolytic removal of 5'-nucleotides from the 3'-hydroxy termini of 3'-hydroxy-terminated oligonucleotides. Relationships: is a type of GO:0004527; is a type of GO:0008081